{
  "term_id": "GO:0000793",
  "gene_symbol": "CDCA2",
  "gene_name": "Cell division cycle-associated protein 2",
  "term_label": "condensed chromosome",
  "gene": "UniProtKB:Q69YH5"
}